{
  "gene_symbol": "MCCC1",
  "gene_name": "Methylcrotonoyl-CoA carboxylase subunit alpha, mitochondrial",
  "gene": "UniProtKB:Q96RQ3",
  "term_id": "GO:0005739",
  "term_label": "mitochondrion"
}